{
  "term_label": "unfolded protein binding",
  "term_id": "GO:0051082",
  "gene_name": "Hsp90 co-chaperone Cdc37-like 1",
  "gene": "UniProtKB:Q7L3B6",
  "gene_symbol": "CDC37L1"
}